{
  "gene_symbol": "CHRNA3",
  "gene_name": "Neuronal acetylcholine receptor subunit alpha-3",
  "term_id": "GO:0005886",
  "term_label": "plasma membrane",
  "gene": "UniProtKB:P32297"
}